{
  "term_label": "Cul3-RING ubiquitin ligase complex",
  "gene_symbol": "KLHL41",
  "gene_name": "Kelch-like protein 41",
  "term_id": "GO:0031463",
  "gene": "UniProtKB:O60662"
}